hydroperoxy icosatetraenoate dehydratase activity [GO:0106256] (MF) References: PMID:12881489 Sources: RHEA:55556 Definition: A hydroperoxy icosatetraenoate = an oxoicosatetraenoate + H2O. Relationships: is a type of hydro-lyase activity [GO:0016836]